benzene biosynthetic process [GO:1900997] (biological process) Also known as: benzene anabolism, benzene biosynthesis, benzene formation, benzene synthesis Relationships: is a type of benzene metabolic process [GO:0018910]; is a type of GO:0120251 Sources: GOC:TermGenie, GOC:yaf, UniPathway:UPA00272 Definition: The chemical reactions and pathways resulting in the formation of benzene.